{
  "gene_symbol": "CCDC24",
  "gene": "UniProtKB:Q8N4L8",
  "gene_name": "Coiled-coil domain-containing protein 24",
  "term_id": "UNKNOWN:0002",
  "term_label": "Unknown biological process"
}